(3R)-(E)-nerolidol synthase activity [GO:0102145] (molecular function) Definition: Catalysis of the reaction: 2-trans,6-trans-farnesyl diphosphate + H2O = (3R,6E)-nerolidol + diphosphoric acid. Sources: GOC:pz, RHEA:27534 Relationships: is a type of carbon-oxygen lyase activity, acting on phosphates [GO:0016838]